{
  "gene": "UniProtKB:P22736",
  "term_label": "cellular response to corticotropin-releasing hormone stimulus",
  "term_id": "GO:0071376",
  "gene_symbol": "NR4A1",
  "gene_name": "Nuclear receptor subfamily 4 group A member 1"
}